{
  "term_id": "GO:0030030",
  "gene": "UniProtKB:Q9P2E2",
  "gene_name": "Kinesin-like protein KIF17",
  "gene_symbol": "KIF17",
  "term_label": "cell projection organization"
}